actin-dependent intracellular transport of virus [GO:0075520] (biological process) Subtypes: GO:0039680 Definition: The directed movement of a virus, or part of a virus, within the host cell cytoplasm via the host's actin filaments. Actin-dependent transport is induced by viral proteins that interact with actin and/or host cell motor proteins like myosins or that promotes actin polymerization/depolymerization reactions. Sources: UniProtKB-KW:KW-1178, VZ:991 Relationships: is_a GO:0075733 Also known as: actin-dependent intracellular transport of viral material